{
  "gene": "UniProtKB:Q5TCZ1",
  "gene_name": "SH3 and PX domain-containing protein 2A",
  "gene_symbol": "SH3PXD2A",
  "term_label": "cytoplasm",
  "term_id": "GO:0005737"
}